{
  "gene": "UniProtKB:Q8TCT6",
  "term_id": "GO:0098554",
  "term_label": "cytoplasmic side of endoplasmic reticulum membrane",
  "gene_name": "Signal peptide peptidase-like 3",
  "gene_symbol": "SPPL3"
}